growth factor dependent regulation of skeletal muscle satellite cell proliferation [GO:0014843] (biological process) References: PMID:16607119 Sources: GOC:ef, GOC:mtg_muscle Definition: Any process that modulates the frequency, rate or extent of satellite cell proliferation; dependent on specific growth factor activity such as fibroblast growth factors and transforming growth factor beta. Relationships: is a type of regulation of skeletal muscle satellite cell proliferation [GO:0014842]